tRNA-intron lyase activity [GO:0000213] (molecular function) Sources: EC:4.6.1.16 Definition: Catalysis of the reaction: pretRNA = a 3'-half-tRNA molecule with a 5'-OH end + a 5'-half-tRNA molecule with a 2',3'-cyclic phosphate end + an intron with a 2',3'-cyclic phosphate and a 5'-hydroxyl terminus. Relationships: is a type of RNA endonuclease activity [GO:0004521]; is a type of GO:0004549; is a type of phosphorus-oxygen lyase activity [GO:0016849] Also known as: tRNA-intron endonuclease activity, tRNA-intron endoribonuclease activity, tRNA splicing endonuclease activity